decylcitrate synthase activity [GO:0050457] (molecular function) Sources: RHEA:16605 Also known as: (2S,3S)-2-hydroxytridecane-1,2,3-tricarboxylate oxaloacetate-lyase (CoA- acylating) activity, (2S,3S)-2-hydroxytridecane-1,2,3-tricarboxylate oxaloacetate-lyase (CoA-acylating), 2-decylcitrate synthase activity, dodecanoyl-CoA:oxaloacetate C-dodecanoyltransferase (thioester-hydrolysing, 1-carboxyundecyl-forming) Definition: Catalysis of the reaction: H2O + lauroyl-CoA + oxaloacetate = (2S,3S)-2-hydroxytridecane-1,2,3-tricarboxylate + CoA + H+. Relationships: is a type of acyltransferase activity, acyl groups converted into alkyl on transfer [GO:0046912]